L-valine transmembrane import into vacuole [GO:0110101] (biological process) Definition: The directed movement of L-valine into the vacuole across the vacuolar membrane. Relationships: is a type of GO:0034491; is a type of L-valine transmembrane transport [GO:1903785] References: PMID:20944394 Sources: GOC:al